{
  "term_label": "Unknown cellular component",
  "gene_name": "Ubiquitin-like protein 3",
  "gene_symbol": "UBL3",
  "term_id": "UNKNOWN:0003",
  "gene": "UniProtKB:O95164"
}